L-xylulose reductase (NADH) activity [GO:0044105] (molecular function) Relationships: is a type of GO:0016616 Definition: Catalysis of the reaction: xylitol + NAD+ = L-xylulose + NADH + H+. References: PMID:14736891 Sources: RHEA:68100